descending thin limb development [GO:0072022] (biological process) Subtypes: GO:0072063, GO:0072064, metanephric descending thin limb development [GO:0072220] Definition: The process whose specific outcome is the progression of the descending thin limb over time, from its formation to the mature structure. The descending thin limb is a part of the loop of Henle situated just after the proximal straight tubule (S3). It extends to the tip of the loop of Henle. Relationships: is_a anatomical structure development [GO:0048856]; is part of loop of Henle development [GO:0072070] Sources: GOC:mtg_kidney_jan10